{
  "gene_name": "Ephrin type-B receptor 2",
  "term_id": "GO:0007411",
  "gene_symbol": "EPHB2",
  "term_label": "axon guidance",
  "gene": "UniProtKB:P29323"
}